{
  "gene": "UniProtKB:P07711",
  "term_id": "GO:0005615",
  "term_label": "extracellular space",
  "gene_name": "Procathepsin L",
  "gene_symbol": "CTSL"
}